{
  "gene_name": "Sialomucin core protein 24",
  "term_id": "GO:0005768",
  "gene_symbol": "CD164",
  "term_label": "endosome",
  "gene": "UniProtKB:Q04900"
}